{
  "term_id": "GO:0035556",
  "gene": "UniProtKB:P20794",
  "gene_name": "Serine_threonine-protein kinase MAK",
  "term_label": "intracellular signal transduction",
  "gene_symbol": "MAK"
}